{
  "gene_symbol": "ZNF480",
  "term_id": "GO:0000978",
  "gene": "UniProtKB:Q8WV37",
  "term_label": "RNA polymerase II cis-regulatory region sequence-specific DNA binding",
  "gene_name": "Zinc finger protein 480"
}